{
  "gene_symbol": "LURAP1L",
  "term_id": "UNKNOWN:0001",
  "term_label": "Unknown molecular function",
  "gene_name": "Leucine rich adaptor protein 1-like",
  "gene": "UniProtKB:Q8IV03"
}